{
  "gene_name": "High affinity immunoglobulin alpha and immunoglobulin mu Fc receptor",
  "gene_symbol": "FCAMR",
  "term_id": "GO:0004888",
  "term_label": "transmembrane signaling receptor activity",
  "gene": "UniProtKB:Q8WWV6"
}